{
  "term_id": "GO:0072384",
  "term_label": "organelle transport along microtubule",
  "gene": "UniProtKB:Q9Y678",
  "gene_symbol": "COPG1",
  "gene_name": "Coatomer subunit gamma-1"
}